{
  "gene": "UniProtKB:Q32P28",
  "gene_name": "Prolyl 3-hydroxylase 1",
  "gene_symbol": "P3H1",
  "term_label": "procollagen-proline 3-dioxygenase activity",
  "term_id": "GO:0019797"
}